{
  "gene_name": "Putative homeobox protein Meis3-like 1",
  "term_id": "GO:0001525",
  "gene_symbol": "MEIS3P1",
  "term_label": "angiogenesis",
  "gene": "UniProtKB:A6NDR6"
}